{
  "term_label": "Unknown biological process",
  "gene_name": "U11_U12 small nuclear ribonucleoprotein 25 kDa protein",
  "gene_symbol": "SNRNP25",
  "term_id": "UNKNOWN:0002",
  "gene": "UniProtKB:Q9BV90"
}